lactone biosynthetic process [GO:1901336] (biological process) Subtypes: L-ascorbic acid biosynthetic process [GO:0019853], GO:0033068, enniatin biosynthetic process [GO:0046585], dehydro-D-arabinono-1,4-lactone biosynthetic process [GO:0070485], GO:0140446, mycophenolic acid biosynthetic process [GO:0140722], GO:0140723, lovastatin biosynthetic process [GO:0140735], paraherquonin biosynthetic process [GO:0140874], mevastatin biosynthetic process [GO:0140877], emericellamide biosynthetic process [GO:1900557], cspyrone B1 biosynthetic process [GO:1900802], (-)-microperfuranone biosynthetic process [GO:1901512], GO:1901601, pentalenolactone biosynthetic process [GO:1901780] Relationships: is_a GO:0009058; is a type of GO:1901334 Also known as: lactone anabolism, lactone biosynthesis, lactone formation, lactone synthesis Definition: The chemical reactions and pathways resulting in the formation of lactone. Sources: GOC:TermGenie